4-hydroxybenzoate 1-hydroxylase activity [GO:0018678] (molecular function) Relationships: is a type of GO:0016709 Definition: Catalysis of the reaction: 4-hydroxybenzoate + NADPH + H+ + O2 = hydroquinone + NADP+ + H2O + CO2. Also known as: 4-hydroxybenzoate 1-monooxygenase activity, 4-hydroxybenzoate,NAD(P)H:oxygen oxidoreductase (1-hydroxylating, decarboxylating) Sources: EC:1.14.13.64